{
  "gene_symbol": "SLC26A3",
  "gene_name": "Chloride anion exchanger",
  "term_id": "GO:0140900",
  "term_label": "chloride:bicarbonate antiporter activity",
  "gene": "UniProtKB:P40879"
}